regulation of mitotic sister chromatid arm separation [GO:1905822] (biological process) Definition: Any process that modulates the frequency, rate or extent of mitotic sister chromatid arm separation. Relationships: is a type of regulation of mitotic sister chromatid separation [GO:0010965]; regulates mitotic sister chromatid arm separation [GO:1990891] Subtypes: GO:1905823, GO:1905824 References: PMID:18765790 Sources: GOC:TermGenie, GOC:als, GO_REF:0000058